{
  "gene": "UniProtKB:P51157",
  "gene_symbol": "RAB28",
  "term_id": "GO:0003924",
  "gene_name": "Ras-related protein Rab-28",
  "term_label": "GTPase activity"
}